{
  "gene": "UniProtKB:Q7KZN9",
  "gene_symbol": "COX15",
  "gene_name": "Cytochrome c oxidase assembly protein COX15 homolog",
  "term_label": "heme A biosynthetic process",
  "term_id": "GO:0006784"
}